{
  "gene_name": "Pescadillo homolog",
  "term_label": "maturation of LSU-rRNA from tricistronic rRNA transcript (SSU-rRNA, 5.8S rRNA, LSU-rRNA)",
  "term_id": "GO:0000463",
  "gene_symbol": "PES1",
  "gene": "UniProtKB:O00541"
}